{
  "term_label": "caspase binding",
  "gene": "UniProtKB:Q13158",
  "gene_symbol": "FADD",
  "term_id": "GO:0089720",
  "gene_name": "FAS-associated death domain protein"
}